negative regulation of calcium ion-dependent exocytosis of neurotransmitter [GO:1903234] (biological process) Relationships: is a type of GO:0045955; is a type of regulation of calcium ion-dependent exocytosis of neurotransmitter [GO:1903233]; is a type of negative regulation of synaptic vesicle exocytosis [GO:2000301]; negatively regulates calcium ion-regulated exocytosis of neurotransmitter [GO:0048791] Also known as: down regulation of calcium ion-dependent exocytosis of neurotransmitter, down-regulation of calcium ion-dependent exocytosis of neurotransmitter, downregulation of calcium ion-dependent exocytosis of neurotransmitter, inhibition of calcium ion-dependent exocytosis of neurotransmitter References: PMID:16782817 Sources: GOC:TermGenie, GO_REF:0000058 Note: An example of this is Rab3gap1 in mouse (Q80UJ7) in PMID:16782817 (IMP) Definition: Any process that stops, prevents or reduces the frequency, rate or extent of calcium ion-dependent exocytosis of neurotransmitter.